{
  "gene_name": "Serine_threonine-protein phosphatase PP1-gamma catalytic subunit",
  "gene": "UniProtKB:P36873",
  "gene_symbol": "PPP1CC",
  "term_label": "regulation of circadian rhythm",
  "term_id": "GO:0042752"
}